{
  "gene_name": "Elongin-C",
  "term_label": "elongin complex",
  "gene_symbol": "ELOC",
  "gene": "UniProtKB:Q15369",
  "term_id": "GO:0070449"
}